regulation of neutrophil differentiation [GO:0045658] (biological process) Subtypes: negative regulation of neutrophil differentiation [GO:0045659], positive regulation of neutrophil differentiation [GO:0045660] Relationships: is a type of GO:0030852; regulates GO:0030223 Sources: GOC:go_curators Definition: Any process that modulates the frequency, rate or extent of neutrophil differentiation.